{
  "gene": "UniProtKB:P52803",
  "gene_symbol": "EFNA5",
  "term_label": "plasma membrane",
  "gene_name": "Ephrin-A5",
  "term_id": "GO:0005886"
}